{
  "term_id": "GO:0035556",
  "term_label": "intracellular signal transduction",
  "gene": "UniProtKB:P56278",
  "gene_name": "Protein p13 MTCP-1",
  "gene_symbol": "MTCP1"
}